{
  "gene_name": "General transcription and DNA repair factor IIH helicase subunit XPB",
  "term_label": "hair cell differentiation",
  "gene_symbol": "ERCC3",
  "gene": "UniProtKB:P19447",
  "term_id": "GO:0035315"
}